{
  "gene": "UniProtKB:Q9NRY7",
  "term_label": "Unknown molecular function",
  "gene_symbol": "PLSCR2",
  "term_id": "UNKNOWN:0001",
  "gene_name": "Phospholipid scramblase 2"
}